{
  "term_id": "GO:0055085",
  "gene": "UniProtKB:P45844",
  "gene_name": "ATP-binding cassette sub-family G member 1",
  "gene_symbol": "ABCG1",
  "term_label": "transmembrane transport"
}